{
  "term_id": "GO:0006303",
  "gene_symbol": "DCLRE1B",
  "gene_name": "5' exonuclease Apollo",
  "gene": "UniProtKB:Q9H816",
  "term_label": "double-strand break repair via nonhomologous end joining"
}